{
  "gene": "UniProtKB:Q8N4T4",
  "term_label": "plasma membrane",
  "term_id": "GO:0005886",
  "gene_name": "Rho guanine nucleotide exchange factor 39",
  "gene_symbol": "ARHGEF39"
}